maintenance of ER location [GO:0051685] (biological process) Sources: GOC:ai, GOC:dph, GOC:tb Definition: Any process in which the endoplasmic reticulum is maintained in a specific location within a cell and prevented from moving elsewhere. Relationships: is a type of endoplasmic reticulum localization [GO:0051643]; is a type of maintenance of organelle location [GO:0051657] Also known as: maintenance of endoplasmic reticulum localization, maintenance of ER localization Subtypes: vacuole-ER tethering [GO:1990854]